{
  "gene_name": "Pre-B-cell leukemia transcription factor 3",
  "term_label": "animal organ morphogenesis",
  "gene_symbol": "PBX3",
  "gene": "UniProtKB:P40426",
  "term_id": "GO:0009887"
}